{
  "gene": "UniProtKB:P02649",
  "term_label": "extracellular vesicle",
  "gene_symbol": "APOE",
  "gene_name": "Apolipoprotein E",
  "term_id": "GO:1903561"
}